{
  "gene_name": "Protein Abitram",
  "term_label": "lamellipodium",
  "term_id": "GO:0030027",
  "gene_symbol": "ABITRAM",
  "gene": "UniProtKB:Q9NX38"
}